{
  "gene": "UniProtKB:A6NNZ2",
  "term_label": "structural constituent of cytoskeleton",
  "gene_symbol": "TUBB8B",
  "gene_name": "Tubulin beta 8B",
  "term_id": "GO:0005200"
}